{
  "gene_symbol": "FSTL5",
  "gene_name": "Follistatin-related protein 5",
  "gene": "UniProtKB:Q8N475",
  "term_id": "UNKNOWN:0001",
  "term_label": "Unknown molecular function"
}